HLH domain binding [GO:0043398] (MF) Sources: GOC:go_curators, Prosite:PDOC0038 Relationships: is a type of GO:0019904 Definition: Binding to a Helix Loop Helix domain, a domain of 40-50 residues that occurs in specific DNA-binding proteins that act as transcription factors. The domain is formed of two amphipathic helices joined by a variable length linker region that can form a loop and it mediates protein dimerization.